{
  "gene_symbol": "PRDM1",
  "term_label": "RNA polymerase II cis-regulatory region sequence-specific DNA binding",
  "term_id": "GO:0000978",
  "gene": "UniProtKB:O75626",
  "gene_name": "PR domain zinc finger protein 1"
}